regulation of pyrimidine nucleotide biosynthetic process [GO:1900397] (BP) Subtypes: GO:1900398, positive regulation of pyrimidine nucleotide biosynthetic process [GO:1900399], regulation of dCDP biosynthetic process [GO:1903528] Also known as: regulation of pyrimidine nucleotide anabolism, regulation of pyrimidine nucleotide biosynthesis, regulation of pyrimidine nucleotide formation, regulation of pyrimidine nucleotide synthesis Relationships: is a type of regulation of nucleotide biosynthetic process [GO:0030808]; regulates GO:0006221 Sources: GOC:TermGenie Definition: Any process that modulates the frequency, rate or extent of pyrimidine nucleotide biosynthetic process.